{
  "term_id": "UNKNOWN:0001",
  "gene": "UniProtKB:P56282",
  "gene_symbol": "POLE2",
  "gene_name": "DNA polymerase epsilon subunit 2",
  "term_label": "Unknown molecular function"
}